{
  "gene": "UniProtKB:O43323",
  "gene_name": "Desert hedgehog protein",
  "term_label": "regulation of gene expression",
  "gene_symbol": "DHH",
  "term_id": "GO:0010468"
}